{
  "term_label": "RNA polymerase II, core complex",
  "gene_name": "DNA-directed RNA polymerase II subunit GRINL1A",
  "term_id": "GO:0005665",
  "gene": "UniProtKB:P0CAP2",
  "gene_symbol": "POLR2M"
}